{
  "term_label": "mitochondrial large ribosomal subunit",
  "term_id": "GO:0005762",
  "gene": "UniProtKB:Q9BYD1",
  "gene_symbol": "MRPL13",
  "gene_name": "Large ribosomal subunit protein uL13m"
}